{
  "gene": "UniProtKB:Q9UNW9",
  "term_label": "mRNA splicing, via spliceosome",
  "term_id": "GO:0000398",
  "gene_symbol": "NOVA2",
  "gene_name": "RNA-binding protein Nova-2"
}